{
  "term_label": "Unknown cellular component",
  "gene_name": "Sterile alpha motif domain-containing protein 3",
  "gene_symbol": "SAMD3",
  "gene": "UniProtKB:Q8N6K7",
  "term_id": "UNKNOWN:0003"
}